{
  "gene": "UniProtKB:Q5YKI7",
  "gene_name": "Putative gametogenetin-binding protein 1",
  "gene_symbol": "GGNBP1",
  "term_id": "UNKNOWN:0002",
  "term_label": "Unknown biological process"
}